negative regulation of central tolerance induction [GO:0002647] (BP) Relationships: is a type of negative regulation of tolerance induction [GO:0002644]; is a type of regulation of central tolerance induction [GO:0002646]; negatively regulates GO:0002508 Definition: Any process that stops, prevents, or reduces the frequency, rate, or extent of central tolerance induction. Also known as: down regulation of central tolerance induction, down-regulation of central tolerance induction, downregulation of central tolerance induction, inhibition of central tolerance induction Sources: GOC:add Subtypes: negative regulation of central B cell tolerance induction [GO:0002896]